dentin mineralization [GO:0097188] (biological process) References: PMID:10206335, PMID:21196346 Sources: GOC:sl Relationships: is a type of tooth mineralization [GO:0034505]; is part of GO:0097187 Also known as: dentine mineralization Definition: The process in which calcium salts are deposited into the calcareous tooth structure known as dentin.